{
  "gene_name": "Alpha-hemoglobin-stabilizing protein",
  "term_label": "erythrocyte differentiation",
  "gene": "UniProtKB:Q9NZD4",
  "gene_symbol": "AHSP",
  "term_id": "GO:0030218"
}